ubiquitin protein ligase activity [GO:0061630] (molecular function) Regulation: regulated by regulation of ubiquitin protein ligase activity [GO:1904666]; negatively regulated by negative regulation of ubiquitin protein ligase activity [GO:1904667]; positively regulated by positive regulation of ubiquitin protein ligase activity [GO:1904668] Definition: Catalysis of the transfer of ubiquitin to a substrate protein via the reaction X-ubiquitin + S = X + S-ubiquitin, where X is either an E2 or E3 enzyme, the X-ubiquitin linkage is a thioester bond, and the S-ubiquitin linkage is an amide bond: an isopeptide bond between the C-terminal glycine of ubiquitin and the epsilon-amino group of lysine residues in the substrate or, in the linear extension of ubiquitin chains, a peptide bond the between the C-terminal glycine and N-terminal methionine of ubiquitin residues. Subtypes: GO:0034450, histone ubiquitin ligase activity [GO:0140852] Also known as: E3, protein ubiquitination activity, ubiquitin ligase activity, ER-associated E3 ligase References: PMID:22863777 Sources: GOC:BioGRID, GOC:dph, GOC:mah, GOC:tb Relationships: is a type of GO:0004842; is a type of ubiquitin-like protein ligase activity [GO:0061659] Note: This enzyme catalyzes a transferase reaction.